{
  "term_label": "cellular response to interferon-beta",
  "gene_symbol": "IFI16",
  "gene_name": "Gamma-interferon-inducible protein 16",
  "gene": "UniProtKB:Q16666",
  "term_id": "GO:0035458"
}